{
  "gene_symbol": "C10orf95",
  "term_id": "UNKNOWN:0003",
  "gene": "UniProtKB:Q9H7T3",
  "term_label": "Unknown cellular component",
  "gene_name": "Uncharacterized protein C10orf95"
}